{
  "gene_symbol": "SPECC1",
  "term_label": "filamentous actin",
  "gene": "UniProtKB:Q5M775",
  "gene_name": "Cytospin-B",
  "term_id": "GO:0031941"
}